{
  "gene": "UniProtKB:Q9HCE5",
  "gene_symbol": "METTL14",
  "term_label": "mRNA binding",
  "term_id": "GO:0003729",
  "gene_name": "N6-adenosine-methyltransferase non-catalytic subunit"
}